{
  "gene_name": "Serine_arginine-rich splicing factor 7",
  "gene": "UniProtKB:Q16629",
  "term_id": "GO:0003729",
  "gene_symbol": "SRSF7",
  "term_label": "mRNA binding"
}